endothelial tip cell filopodium assembly [GO:0120084] (biological process) Definition: The assembly of a filopodium, a thin, stiff protrusion extended by the endothelial tip cell of a vascular sprout. References: PMID:28264837 Sources: GOC:cvs Relationships: is a type of filopodium assembly [GO:0046847]